{
  "gene_symbol": "AP1S2",
  "gene": "UniProtKB:P56377",
  "gene_name": "AP-1 complex subunit sigma-2",
  "term_id": "GO:0016192",
  "term_label": "vesicle-mediated transport"
}